{
  "gene_name": "Suppressor of tumorigenicity 14 protein",
  "term_label": "plasma membrane",
  "term_id": "GO:0005886",
  "gene": "UniProtKB:Q9Y5Y6",
  "gene_symbol": "ST14"
}